{
  "gene_name": "Enhancer of filamentation 1",
  "gene_symbol": "NEDD9",
  "gene": "UniProtKB:Q14511",
  "term_id": "UNKNOWN:0001",
  "term_label": "Unknown molecular function"
}